{
  "gene_symbol": "RGMB",
  "term_id": "GO:0005886",
  "gene_name": "Repulsive guidance molecule B",
  "gene": "UniProtKB:Q6NW40",
  "term_label": "plasma membrane"
}